{
  "term_id": "GO:0004674",
  "gene_symbol": "TTBK1",
  "term_label": "protein serine/threonine kinase activity",
  "gene_name": "Tau-tubulin kinase 1",
  "gene": "UniProtKB:Q5TCY1"
}